{
  "gene_symbol": "IQGAP1",
  "term_label": "nucleus",
  "gene": "UniProtKB:P46940",
  "gene_name": "Ras GTPase-activating-like protein IQGAP1",
  "term_id": "GO:0005634"
}